regulation of fever generation [GO:0031620] (biological process) Sources: GOC:add, GOC:dph, GOC:tb Relationships: is a type of regulation of acute inflammatory response [GO:0002673]; is a type of regulation of heat generation [GO:0031650]; regulates fever generation [GO:0001660] Definition: Any process that modulates the rate or extent of fever generation. Also known as: regulation of pyrexia Subtypes: negative regulation of fever generation [GO:0031621], positive regulation of fever generation [GO:0031622], GO:0071809, regulation of fever generation by regulation of prostaglandin secretion [GO:0071810]